maintenance of meiotic sister chromatid cohesion, centromeric [GO:0035875] (biological process) Relationships: is a type of maintenance of meiotic sister chromatid cohesion [GO:0034090]; is part of meiotic sister chromatid cohesion, centromeric [GO:0051754] Subtypes: GO:1990813 Definition: The process in which the association between sister chromatids of a replicated chromosome along the length of the centromeric region is maintained as chromosomes condense, attach to the spindle in a bipolar orientation, and congress to the metaphase plate during a meiotic cell cycle. Regulation: regulated by regulation of maintenance of meiotic sister chromatid cohesion, centromeric [GO:2000709]; negatively regulated by GO:2000710; positively regulated by positive regulation of maintenance of meiotic sister chromatid cohesion, centromeric [GO:2000711] References: PMID:1708436 Sources: GOC:vw Also known as: maintenance of centromeric meiotic sister chromatin cohesion, maintenance of meiotic sister chromatin cohesion at centromere, maintenance of sister chromatin cohesion at centromere at meiosis I